{
  "gene": "UniProtKB:P52744",
  "gene_symbol": "ZNF138",
  "term_label": "regulation of DNA-templated transcription",
  "gene_name": "Zinc finger protein 138",
  "term_id": "GO:0006355"
}